{
  "gene_symbol": "HBB",
  "term_label": "hemoglobin complex",
  "gene_name": "Hemoglobin subunit beta",
  "term_id": "GO:0005833",
  "gene": "UniProtKB:P68871"
}